has_exact_synonym [oboInOwl#hasExactSynonym]